eukaryotic 80S initiation complex [GO:0033291] (cellular component) Relationships: is a type of translation initiation complex [GO:0070992] Definition: A protein complex composed of the large and small ribosomal subunits, methionyl-initiatior tRNA, and the capped mRNA. The initiator tRNA is positioned at the ribosomal P site at the AUG codon corresponding to the beginning of the coding region. References: PMID:15145049 Sources: GOC:hjd